{
  "term_label": "cyclin-dependent protein serine/threonine kinase inhibitor activity",
  "gene_name": "Cyclin-dependent kinase inhibitor 2A",
  "gene": "UniProtKB:P42771",
  "term_id": "GO:0004861",
  "gene_symbol": "CDKN2A"
}